cell adhesion involved in amphid sensory organ dendrite retrograde extension [GO:0003396] (biological process) Definition: The directed, self-propelled movement of a neuron that contributes to the process of retrograde extension of a dendrite in a neuron of the amphid sensory organ. Relationships: is a type of cell adhesion involved in dendrite retrograde extension [GO:0003394]; is part of amphid sensory organ dendrite retrograde extension [GO:0003391] Sources: GOC:ascb_2009, GOC:dph, GOC:tb